{
  "term_label": "nucleus",
  "term_id": "GO:0005634",
  "gene": "UniProtKB:Q59H18",
  "gene_symbol": "TNNI3K",
  "gene_name": "Serine_threonine-protein kinase TNNI3K"
}